{
  "gene_name": "Membrane-associated phosphatidylinositol transfer protein 1",
  "gene": "UniProtKB:O00562",
  "term_id": "GO:0035091",
  "term_label": "phosphatidylinositol binding",
  "gene_symbol": "PITPNM1"
}